{
  "gene_name": "Cysteine dioxygenase type 1",
  "gene": "UniProtKB:Q16878",
  "term_label": "Unknown cellular component",
  "term_id": "UNKNOWN:0003",
  "gene_symbol": "CDO1"
}